cholesterol storage [GO:0010878] (biological process) Regulation: regulated by regulation of cholesterol storage [GO:0010885]; positively regulated by GO:0010886; negatively regulated by negative regulation of cholesterol storage [GO:0010887] Relationships: is a type of lipid storage [GO:0019915] Also known as: cholesterol sequestration, sequestration of cholesterol Definition: The accumulation and maintenance in cells or tissues of cholesterol, cholest-5-en-3 beta-ol, the principal sterol of vertebrates and the precursor of many steroids, including bile acids and steroid hormones. Sources: GOC:BHF, GOC:dph, GOC:tb